{
  "term_label": "cytokine-mediated signaling pathway",
  "gene": "UniProtKB:O14543",
  "gene_symbol": "SOCS3",
  "gene_name": "Suppressor of cytokine signaling 3",
  "term_id": "GO:0019221"
}